protein insertion into mitochondrial inner membrane from matrix [GO:0032979] (biological process) References: PMID:12880202, PMID:15473843 Sources: GOC:vw Definition: The process in which a protein is incorporated into the mitochondrial inner membrane from the matrix side. This includes membrane insertion of newly synthesized mitochondrially-encoded proteins, and insertion of nuclear-encoded proteins after their import into the mitochondrial matrix. Also known as: insertion of proteins into the mitochondrial membrane from the inner side, protein insertion into mitochondrial inner membrane from matrix side, protein insertion into mitochondrial membrane from inner side Relationships: is a type of protein insertion into mitochondrial inner membrane [GO:0045039]